flavin adenine dinucleotide binding [GO:0050660] (MF) Subtypes: FAD binding [GO:0071949], GO:0071950 Relationships: is a type of nucleotide binding [GO:0000166]; is a type of anion binding [GO:0043168] Also known as: FAD or FADH2 binding, flavine-adenine dinucleotide binding Definition: Binding to FAD, flavin-adenine dinucleotide, the coenzyme or the prosthetic group of various flavoprotein oxidoreductase enzymes, in either the oxidized form, FAD, or the reduced form, FADH2. Sources: GOC:ai, GOC:imk, ISBN:0198506732